{
  "gene_symbol": "CCN5",
  "gene": "UniProtKB:O76076",
  "term_label": "extracellular space",
  "term_id": "GO:0005615",
  "gene_name": "CCN family member 5"
}